{
  "term_label": "Unknown biological process",
  "gene": "UniProtKB:Q5T7P2",
  "term_id": "UNKNOWN:0002",
  "gene_name": "Late cornified envelope protein 1A",
  "gene_symbol": "LCE1A"
}